{
  "gene": "UniProtKB:Q9BYR4",
  "gene_symbol": "KRTAP4-3",
  "term_label": "hair cycle",
  "term_id": "GO:0042633",
  "gene_name": "Keratin-associated protein 4-3"
}